phosphatidylglycerol-membrane-oligosaccharide glycerophosphotransferase activity [GO:0008960] (molecular function) Also known as: oligosaccharide glycerophosphotransferase activity, phosphatidylglycerol:membrane-derived-oligosaccharide-D-glucose glycerophosphotransferase activity, phosphoglycerol transferase I, phosphoglycerol transferase activity Relationships: is a type of phosphotransferase activity, for other substituted phosphate groups [GO:0016780] Sources: EC:2.7.8.20 Definition: Catalysis of the reaction: phosphatidylglycerol + membrane-derived-oligosaccharide D-glucose = 1,2-diacyl-sn-glycerol + membrane-derived-oligosaccharide 6-(glycerophospho)-D-glucose.